{
  "gene": "UniProtKB:Q9NXG0",
  "term_id": "UNKNOWN:0001",
  "term_label": "Unknown molecular function",
  "gene_symbol": "CNTLN",
  "gene_name": "Centlein"
}